regulation of glycolytic process through fructose-6-phosphate [GO:1904538] (biological process) Subtypes: negative regulation of glycolytic process through fructose-6-phosphate [GO:1904539], positive regulation of glycolytic process through fructose-6-phosphate [GO:1904540] Definition: Any process that modulates the frequency, rate or extent of glycolytic process through fructose-6-phosphate. Sources: GOC:TermGenie, GOC:dph, GO_REF:0000058, ISBN:0201090910, ISBN:0879010479 Also known as: regulation of glycolysis through fructose-6-phosphate Relationships: is a type of GO:0006110; regulates glycolytic process through fructose-6-phosphate [GO:0061615]